{
  "gene_symbol": "MYO5B",
  "gene_name": "Unconventional myosin-Vb",
  "term_id": "GO:0051015",
  "gene": "UniProtKB:Q9ULV0",
  "term_label": "actin filament binding"
}